TMP biosynthetic process [GO:0006230] (biological process) Definition: The chemical reactions and pathways resulting in the formation of TMP, ribosylthymine monophosphate. Relationships: is a type of GO:0009174; is a type of pyrimidine ribonucleotide biosynthetic process [GO:0009220]; is a type of TMP metabolic process [GO:0046044] Sources: ISBN:0198506732 Also known as: TMP anabolism, TMP biosynthesis, TMP formation, TMP synthesis